{
  "gene_symbol": "MYO9A",
  "gene_name": "Unconventional myosin-IXa",
  "gene": "UniProtKB:B2RTY4",
  "term_id": "GO:0045198",
  "term_label": "establishment of epithelial cell apical/basal polarity"
}